{
  "term_label": "extracellular space",
  "gene_name": "Acid sphingomyelinase-like phosphodiesterase 3a",
  "gene": "UniProtKB:Q92484",
  "gene_symbol": "SMPDL3A",
  "term_id": "GO:0005615"
}